{
  "term_id": "GO:0004722",
  "term_label": "protein serine/threonine phosphatase activity",
  "gene_name": "Serine_threonine-protein phosphatase PP1-beta catalytic subunit",
  "gene_symbol": "PPP1CB",
  "gene": "UniProtKB:P62140"
}